{
  "gene": "UniProtKB:Q96HJ3",
  "gene_symbol": "CCDC34",
  "term_label": "Unknown cellular component",
  "term_id": "UNKNOWN:0003",
  "gene_name": "Coiled-coil domain-containing protein 34"
}